{
  "gene_symbol": "HNRNPK",
  "term_label": "nucleus",
  "gene_name": "Heterogeneous nuclear ribonucleoprotein K",
  "gene": "UniProtKB:P61978",
  "term_id": "GO:0005634"
}